{
  "gene_symbol": "RTTN",
  "term_label": "centriole-centriole cohesion",
  "gene": "UniProtKB:Q86VV8",
  "term_id": "GO:0010457",
  "gene_name": "Rotatin"
}